{
  "term_id": "UNKNOWN:0003",
  "gene_name": "Proline-rich protein 20C",
  "gene": "UniProtKB:P86479",
  "gene_symbol": "PRR20C",
  "term_label": "Unknown cellular component"
}